{
  "gene": "UniProtKB:P37288",
  "gene_name": "Vasopressin V1a receptor",
  "gene_symbol": "AVPR1A",
  "term_id": "GO:0001992",
  "term_label": "regulation of systemic arterial blood pressure by vasopressin"
}